{
  "gene_symbol": "POLD3",
  "gene": "UniProtKB:Q15054",
  "gene_name": "DNA polymerase delta subunit 3",
  "term_id": "GO:0006271",
  "term_label": "DNA strand elongation involved in DNA replication"
}